{
  "gene_symbol": "GPR162",
  "term_label": "Unknown molecular function",
  "gene": "UniProtKB:Q16538",
  "gene_name": "Probable G-protein coupled receptor 162",
  "term_id": "UNKNOWN:0001"
}